{
  "term_id": "UNKNOWN:0002",
  "gene": "UniProtKB:Q5T6F2",
  "gene_symbol": "UBAP2",
  "term_label": "Unknown biological process",
  "gene_name": "Ubiquitin-associated protein 2"
}